N-terminal protein palmitoylation [GO:0006500] (biological process) Relationships: is a type of N-terminal protein lipidation [GO:0006498]; is a type of GO:0018345 Regulation: regulated by GO:0060254; negatively regulated by negative regulation of N-terminal protein palmitoylation [GO:0060262] Sources: GOC:mah Subtypes: N-terminal peptidyl-L-cysteine N-palmitoylation [GO:0018009] Definition: The covalent attachment of a palmitoyl group to the N-terminal amino acid residue of a protein.